{
  "gene_symbol": "PDCD11",
  "gene_name": "Protein RRP5 homolog",
  "term_id": "GO:0032040",
  "gene": "UniProtKB:Q14690",
  "term_label": "small-subunit processome"
}